{
  "gene": "UniProtKB:Q8WX94",
  "gene_name": "NACHT, LRR and PYD domains-containing protein 7",
  "term_id": "GO:0032691",
  "term_label": "negative regulation of interleukin-1 beta production",
  "gene_symbol": "NLRP7"
}